regulation of austinol biosynthetic process [GO:1900640] (biological process) Sources: GOC:TermGenie, GOC:di Relationships: is_a GO:0009889; regulates austinol biosynthetic process [GO:1900560] Definition: Any process that modulates the frequency, rate or extent of austinol biosynthetic process. Also known as: regulation of austinol anabolism, regulation of austinol biosynthesis, regulation of austinol formation, regulation of austinol synthesis Subtypes: negative regulation of austinol biosynthetic process [GO:1900641], positive regulation of austinol biosynthetic process [GO:1900642]